{
  "gene_name": "Leucine-rich repeat-containing protein 25",
  "term_label": "Unknown molecular function",
  "gene_symbol": "LRRC25",
  "gene": "UniProtKB:Q8N386",
  "term_id": "UNKNOWN:0001"
}